biotin synthase activity [GO:0004076] (MF) Relationships: is a type of sulfurtransferase activity [GO:0016783] Definition: Catalysis of the reaction: (4R,5S)-dethiobiotin + [sulfur carrier]-SH + 2 reduced [2Fe-2S]-[ferredoxin] + 2 S-adenosyl-L-methionine = [sulfur carrier]-H + biotin + 2 5'-deoxyadenosine + 2 L-methionine + 2 oxidized [2Fe-2S]-[ferredoxin]. Sources: EC:2.8.1.6, RHEA:22060 Also known as: biotin synthetase activity, dethiobiotin:sulfur sulfurtransferase activity